protein stabilization [GO:0050821] (BP) Also known as: positive regulation of protein stability, protein stabilisation, lysosomal protein stabilization, protein sequestering, protein stabilization activity Sources: GOC:ai Definition: Any process involved in maintaining the structure and integrity of a protein and preventing it from degradation or aggregation. Relationships: is a type of regulation of protein stability [GO:0031647]